negative regulation of apolipoprotein A-I-mediated signaling pathway [GO:1905095] (BP) Also known as: down regulation of apolipoprotein A-I-mediated signaling pathway, down regulation of apolipoprotein A-I-mediated signalling pathway, down-regulation of apolipoprotein A-I-mediated signaling pathway, down-regulation of apolipoprotein A-I-mediated signalling pathway, downregulation of apolipoprotein A-I-mediated signaling pathway, downregulation of apolipoprotein A-I-mediated signalling pathway, negative regulation of apolipoprotein A-I-mediated signalling pathway, inhibition of apolipoprotein A-I-mediated signaling pathway, inhibition of apolipoprotein A-I-mediated signalling pathway References: PMID:25084135 Sources: GOC:BHF, GOC:BHF_miRNA, GOC:TermGenie, GOC:bc, GO_REF:0000058 Definition: Any process that stops, prevents or reduces the frequency, rate or extent of apolipoprotein A-I-mediated signaling pathway. Relationships: is a type of negative regulation of signal transduction [GO:0009968]; is a type of GO:1905094; negatively regulates apolipoprotein A-I-mediated signaling pathway [GO:0038027]